somatic spine [GO:0097465] (cellular component) Sources: NIF_Subcellular:sao2048514053 Relationships: is_a neuron spine [GO:0044309] Definition: Spine emanating from the cell soma of a neuron.